optic nerve morphogenesis [GO:0021631] (biological process) Definition: The process in which the anatomical structure of the optic nerve is generated and organized. The sensory optic nerve originates from the bipolar cells of the retina and conducts visual information to the brainstem. The optic nerve exits the back of the eye in the orbit, enters the optic canal, and enters the central nervous system at the optic chiasm (crossing) where the nerve fibers become the optic tract just prior to entering the hindbrain. Sources: GOC:cls, GOC:dgh, GOC:dph, GOC:jid, GO_REF:0000021 Also known as: CN II morphogenesis Relationships: is a type of cranial nerve morphogenesis [GO:0021602]; is part of optic nerve development [GO:0021554]